amyloid precursor protein catabolic process [GO:0042987] (biological process) Relationships: is a type of amyloid precursor protein metabolic process [GO:0042982] Regulation: regulated by regulation of amyloid precursor protein catabolic process [GO:1902991]; negatively regulated by GO:1902992; positively regulated by GO:1902993 Subtypes: amyloid-beta formation [GO:0034205] Sources: GOC:go_curators Definition: The chemical reactions and pathways resulting in the breakdown of amyloid precursor protein (APP), the precursor of amyloid-beta, a glycoprotein associated with Alzheimer's disease. Also known as: APP catabolic process, APP catabolism, amyloid precursor protein breakdown, amyloid precursor protein catabolism, amyloid precursor protein degradation